{
  "gene_symbol": "TACC1",
  "term_id": "GO:0007097",
  "term_label": "nuclear migration",
  "gene_name": "Transforming acidic coiled-coil-containing protein 1",
  "gene": "UniProtKB:O75410"
}